{
  "gene_symbol": "PORCN",
  "term_id": "GO:0005783",
  "term_label": "endoplasmic reticulum",
  "gene_name": "Protein-serine O-palmitoleoyltransferase porcupine",
  "gene": "UniProtKB:Q9H237"
}